micropexophagy-specific membrane apparatus [GO:0032046] (cellular component) Relationships: is_a GO:0031984; is part of vacuole [GO:0005773] Also known as: MIPA, micropexophagic apparatus References: PMID:15563611 Definition: A membrane-bounded flattened sac that is formed during micropexophagy between the membrane tips of an engulfing vacuole, completing the engulfment and sequestration of peroxisomes from the cytosol, and forming a micropexophagic body within the lumen of the vacuole.